maintenance of protein complex location in cytoplasm [GO:0098545] (biological process) Sources: GOC:dos Relationships: is a type of maintenance of location in cell [GO:0051651]; is a type of maintenance of protein complex location [GO:0098544]; occurs in cytoplasm [GO:0005737] Definition: Any process in which a protein complex is maintained in a specific location within the cytoplasm and is prevented from moving elsewhere.